eukaryotic 43S preinitiation complex [GO:0016282] (cellular component) References: PMID:15145049, PMID:16510876, PMID:25742741, PMID:29735639 Sources: GOC:hjd Definition: A protein complex composed of the 40S ribosomal subunit plus eIF1, eIF1A, eIF3, eIF5, and eIF2-GTP-bound methionyl-initiator methionine tRNA. Relationships: is a type of GO:0070993; has part cytosolic small ribosomal subunit [GO:0022627] Also known as: eukaryotic 43S pre-initiation complex